{
  "term_id": "GO:0120212",
  "term_label": "sperm head-tail coupling apparatus",
  "gene": "UniProtKB:Q8TBY8",
  "gene_name": "Polyamine-modulated factor 1-binding protein 1",
  "gene_symbol": "PMFBP1"
}